{
  "gene_name": "Thioredoxin domain-containing protein 5",
  "term_id": "GO:0003756",
  "term_label": "protein disulfide isomerase activity",
  "gene_symbol": "TXNDC5",
  "gene": "UniProtKB:Q8NBS9"
}